{
  "gene_symbol": "MX2",
  "term_id": "GO:0045202",
  "gene_name": "Interferon-induced GTP-binding protein Mx2",
  "gene": "UniProtKB:P20592",
  "term_label": "synapse"
}